{
  "term_label": "intracellular protein transport",
  "gene_name": "Syntaxin-6",
  "term_id": "GO:0006886",
  "gene": "UniProtKB:O43752",
  "gene_symbol": "STX6"
}